{
  "gene_name": "Phosphatidylinositol 3,4,5-trisphosphate-dependent Rac exchanger 2 protein",
  "term_id": "GO:0005886",
  "gene": "UniProtKB:Q70Z35",
  "term_label": "plasma membrane",
  "gene_symbol": "PREX2"
}